{
  "gene": "UniProtKB:Q6UB98",
  "term_id": "UNKNOWN:0002",
  "term_label": "Unknown biological process",
  "gene_symbol": "ANKRD12",
  "gene_name": "Ankyrin repeat domain-containing protein 12"
}